{
  "gene_name": "Golgin subfamily A member 8K",
  "gene": "UniProtKB:D6RF30",
  "gene_symbol": "GOLGA8K",
  "term_label": "cis-Golgi network",
  "term_id": "GO:0005801"
}